{
  "term_label": "CCR chemokine receptor binding",
  "term_id": "GO:0048020",
  "gene_name": "C-C motif chemokine 1",
  "gene_symbol": "CCL1",
  "gene": "UniProtKB:P22362"
}